{
  "term_label": "signal transduction",
  "term_id": "GO:0007165",
  "gene_symbol": "OLFML2B",
  "gene": "UniProtKB:Q68BL8",
  "gene_name": "Olfactomedin-like protein 2B"
}